{
  "gene_name": "Gamma-secretase subunit PEN-2",
  "term_id": "GO:0007220",
  "gene_symbol": "PSENEN",
  "gene": "UniProtKB:Q9NZ42",
  "term_label": "Notch receptor processing"
}